{
  "term_label": "Unknown cellular component",
  "gene_symbol": "MMD2",
  "term_id": "UNKNOWN:0003",
  "gene_name": "Monocyte to macrophage differentiation factor 2",
  "gene": "UniProtKB:Q8IY49"
}